{
  "term_id": "GO:0005925",
  "term_label": "focal adhesion",
  "gene_name": "Thyroid receptor-interacting protein 6",
  "gene_symbol": "TRIP6",
  "gene": "UniProtKB:Q15654"
}